{
  "gene": "UniProtKB:A0A075B6Z2",
  "gene_name": "T cell receptor alpha joining 56 (Fragment)",
  "gene_symbol": "TRAJ56",
  "term_label": "Unknown biological process",
  "term_id": "UNKNOWN:0002"
}